{
  "gene": "UniProtKB:O95295",
  "gene_name": "SNARE-associated protein Snapin",
  "term_id": "GO:0000149",
  "term_label": "SNARE binding",
  "gene_symbol": "SNAPIN"
}